{
  "gene_name": "17-beta-hydroxysteroid dehydrogenase type 1",
  "term_id": "GO:0005829",
  "term_label": "cytosol",
  "gene": "UniProtKB:P14061",
  "gene_symbol": "HSD17B1"
}